{
  "term_id": "UNKNOWN:0003",
  "gene_name": "Putative uncharacterized protein LOC388882",
  "gene_symbol": "Q8N402",
  "term_label": "Unknown cellular component",
  "gene": "UniProtKB:Q8N402"
}